removal of RNA primer involved in mitotic DNA replication [GO:1903469] (biological process) Relationships: is a type of DNA replication, removal of RNA primer [GO:0043137]; is a type of mitotic cell cycle process [GO:1903047]; is part of mitotic DNA replication [GO:1902969] Definition: Any DNA replication, removal of RNA primer that is involved in mitotic cell cycle DNA replication. References: PMID:1234 Sources: GOC:TermGenie, GOC:mtg_cell_cycle, GO_REF:0000060 Also known as: DNA replication, removal of RNA primer involved in DNA replication involved in S phase involved in mitotic cell cycle, DNA replication, removal of RNA primer involved in DNA replication involved in S-phase involved in mitotic cell cycle, DNA replication, removal of RNA primer involved in mitotic nuclear cell cycle DNA replication, Okazaki initiator RNA removal involved in DNA replication involved in S phase involved in mitotic cell cycle, Okazaki initiator RNA removal involved in DNA replication involved in S-phase involved in mitotic cell cycle, Okazaki initiator RNA removal involved in mitotic cell cycle DNA replication, Okazaki initiator RNA removal involved in mitotic nuclear cell cycle DNA replication, DNA replication, removal of RNA primer involved in DNA replication during S phase involved in mitotic cell cycle, DNA replication, removal of RNA primer involved in nuclear cell cycle DNA replication involved in mitotic cell cycle, Okazaki initiator RNA removal involved in DNA replication during S phase involved in mitotic cell cycle, Okazaki initiator RNA removal involved in nuclear cell cycle DNA replication involved in mitotic cell cycle